{
  "gene": "UniProtKB:Q96JB5",
  "term_label": "endoplasmic reticulum unfolded protein response",
  "term_id": "GO:0030968",
  "gene_name": "CDK5 regulatory subunit-associated protein 3",
  "gene_symbol": "CDK5RAP3"
}